{
  "term_id": "GO:0050911",
  "gene_symbol": "OR2A4",
  "gene": "UniProtKB:O95047",
  "gene_name": "Olfactory receptor 2A4",
  "term_label": "detection of chemical stimulus involved in sensory perception of smell"
}